{
  "term_label": "AMP deaminase activity",
  "gene_symbol": "AMPD1",
  "term_id": "GO:0003876",
  "gene": "UniProtKB:P23109",
  "gene_name": "AMP deaminase 1"
}